protein deacetylation [GO:0006476] (biological process) Relationships: is a type of protein deacylation [GO:0035601] Regulation: regulated by regulation of protein deacetylation [GO:0090311]; positively regulated by positive regulation of protein deacetylation [GO:0090312] Also known as: protein amino acid deacetylation Definition: The removal of an acetyl group from a protein amino acid. An acetyl group is CH3CO-, derived from acetic [ethanoic] acid. Subtypes: peptidyl-lysine deacetylation [GO:0034983], Hsp90 deacetylation [GO:0070846], tubulin deacetylation [GO:0090042] Sources: GOC:ai